stilbene catabolic process [GO:0046272] (biological process) Also known as: stilbene breakdown, stilbene catabolism, stilbene degradation Sources: GOC:ai Definition: The chemical reactions and pathways resulting in the breakdown of stilbenes, a class of polyketide compounds formed from cinnamic acid and three molecules of malonyl CoA. Relationships: is a type of benzene-containing compound metabolic process [GO:0042537]; is a type of GO:0120256